{
  "gene_symbol": "RAB40B",
  "gene": "UniProtKB:Q12829",
  "gene_name": "Ras-related protein Rab-40B",
  "term_label": "GTPase activity",
  "term_id": "GO:0003924"
}